hyponitrite reductase (NADH) activity [GO:0047999] (molecular function) Also known as: NADH2:hyponitrite oxidoreductase activity, NADH:hyponitrite oxidoreductase activity, hydroxylamine:NAD+ oxidoreductase activity Relationships: is a type of oxidoreductase activity, acting on other nitrogenous compounds as donors, with NAD or NADP as acceptor [GO:0046857] Definition: Catalysis of the reaction: 2 hydroxylamine + 2 NAD+ = 2 H+ + hyponitrous acid + 2 NADH. Sources: RHEA:19337